{
  "term_label": "cellular response to fatty acid",
  "gene_name": "Free fatty acid receptor 2",
  "gene": "UniProtKB:O15552",
  "gene_symbol": "FFAR2",
  "term_id": "GO:0071398"
}